{
  "gene_symbol": "IFNK",
  "term_label": "B cell activation involved in immune response",
  "gene": "UniProtKB:Q9P0W0",
  "term_id": "GO:0002312",
  "gene_name": "Interferon kappa"
}